insulin receptor activity [GO:0005009] (molecular function) Also known as: insulin-activated receptor activity Definition: Combining with insulin receptor ligand and transmitting the signal across the plasma membrane to initiate a change in cell activity. Relationships: is_a GO:0004714; is a type of GO:0016500; is part of GO:0008286; has part insulin binding [GO:0043559] Sources: ISBN:0198506732